positive regulation of DNA damage checkpoint [GO:2000003] (biological process) Sources: GOC:obol Also known as: positive regulation of DNA damage response, signal transduction resulting in cell cycle arrest Subtypes: positive regulation of mitotic DNA damage checkpoint [GO:1904291] Definition: Any process that activates or increases the frequency, rate or extent of a DNA damage checkpoint. Relationships: is a type of positive regulation of cell cycle checkpoint [GO:1901978]; is a type of regulation of DNA damage checkpoint [GO:2000001]; positively regulates DNA damage checkpoint signaling [GO:0000077]